{
  "gene_name": "Transcription factor GATA-4",
  "term_id": "GO:0000978",
  "gene": "UniProtKB:P43694",
  "gene_symbol": "GATA4",
  "term_label": "RNA polymerase II cis-regulatory region sequence-specific DNA binding"
}